{
  "term_label": "peptide cross-linking",
  "gene_name": "Protein-glutamine gamma-glutamyltransferase 4",
  "term_id": "GO:0018149",
  "gene": "UniProtKB:P49221",
  "gene_symbol": "TGM4"
}